regulation of secondary metabolite biosynthetic process [GO:1900376] (biological process) Definition: Any process that modulates the frequency, rate or extent of secondary metabolite biosynthetic process. Sources: GOC:TermGenie, GOC:di Relationships: is a type of GO:0009889; is a type of GO:0043455; regulates secondary metabolite biosynthetic process [GO:0044550] Subtypes: regulation of sterigmatocystin biosynthetic process [GO:0010913], regulation of melanin biosynthetic process [GO:0048021], GO:1900177, regulation of penicillin biosynthetic process [GO:1900196], negative regulation of secondary metabolite biosynthetic process [GO:1900377], positive regulation of secondary metabolite biosynthetic process [GO:1900378], regulation of asperthecin biosynthetic process [GO:1900379], regulation of arugosin biosynthetic process [GO:1900626], GO:1900649, regulation of demethylkotanin biosynthetic process [GO:1900652], regulation of diorcinol biosynthetic process [GO:1900655], regulation of emericellamide biosynthetic process [GO:1900658], regulation of emodin biosynthetic process [GO:1900664], regulation of endocrocin biosynthetic process [GO:1900667], regulation of fumonisin biosynthetic process [GO:1900683], GO:1900686, GO:1900689, regulation of (+)-kotanin biosynthetic process [GO:1900692], regulation of N',N'',N'''-triacetylfusarinine C biosynthetic process [GO:1900695], regulation of o-orsellinic acid biosynthetic process [GO:1900698], regulation of orcinol biosynthetic process [GO:1900701], regulation of siderophore biosynthetic process [GO:1900704], regulation of tensidol A biosynthetic process [GO:1900707], GO:1900710, regulation of violaceol I biosynthetic process [GO:1900713], regulation of violaceol II biosynthetic process [GO:1900716], GO:1900732, regulation of ergot alkaloid biosynthetic process [GO:1900822], GO:1900834, regulation of helvolic acid biosynthetic process [GO:1900840], GO:1900843, regulation of cordyol C biosynthetic process [GO:1900861], regulation of lignin biosynthetic process [GO:1901141], GO:1903085, GO:2000029 Also known as: regulation of secondary metabolite biosynthesis